{
  "term_label": "flavin adenine dinucleotide binding",
  "gene_name": "Peroxisomal acyl-coenzyme A oxidase 2",
  "gene": "UniProtKB:Q99424",
  "gene_symbol": "ACOX2",
  "term_id": "GO:0050660"
}